{
  "term_id": "UNKNOWN:0002",
  "gene": "UniProtKB:Q8NGP2",
  "term_label": "Unknown biological process",
  "gene_name": "Olfactory receptor 8J1",
  "gene_symbol": "OR8J1"
}